aldose beta-D-fructosyltransferase activity [GO:0047642] (MF) Definition: Catalysis of the reaction: alpha-D-aldosyl1 beta-D-fructoside + D-aldose2 = D-aldose1 + alpha-D-aldosyl2 beta-D-fructoside. Also known as: aldose b-D-fructosyltransferase activity, alpha-D-aldosyl-beta-D-fructoside:aldose 1-beta-D-fructosyltransferase activity Relationships: is_a GO:0050738 Sources: EC:2.4.1.162, MetaCyc:ALDOSE-BETA-FRUCTOSYLTRANSFERASE-RXN